{
  "gene_symbol": "FRMPD2",
  "gene": "UniProtKB:Q68DX3",
  "gene_name": "FERM and PDZ domain-containing protein 2",
  "term_label": "cytoplasm",
  "term_id": "GO:0005737"
}